{
  "gene": "UniProtKB:Q9UGN5",
  "gene_name": "Poly [ADP-ribose] polymerase 2",
  "term_id": "GO:0003950",
  "term_label": "NAD+ poly-ADP-ribosyltransferase activity",
  "gene_symbol": "PARP2"
}